{
  "term_label": "chromatin",
  "gene": "UniProtKB:Q13148",
  "gene_name": "TAR DNA-binding protein 43",
  "term_id": "GO:0000785",
  "gene_symbol": "TARDBP"
}